{
  "term_label": "centrosome",
  "gene": "UniProtKB:O94986",
  "gene_symbol": "CEP152",
  "term_id": "GO:0005813",
  "gene_name": "Centrosomal protein of 152 kDa"
}